GDP-Man:Man(2)GlcNAc(2)-PP-Dol alpha-1,6-mannosyltransferase activity [GO:0102704] (molecular function) Sources: RHEA:29519 Relationships: is a type of alpha-1,6-mannosyltransferase activity [GO:0000009]; is a type of GlcNAc(2)-PP-Dol mannosyltransferase activity [GO:0120562] Definition: Catalysis of the reaction: an alpha-D-Man-(1->3)-beta-D-Man-(1->4)-beta-D-GlcNAc-(1->4)-alpha-D-GlcNAc-diphospho-di-trans,poly-cis-dolichol + GDP-alpha-D-mannose = an alpha-D-Man-(1->3)-[alpha-D-Man-(1->6)]-beta-D-Man-(1->4)-beta-D-GlcNAc-(1->4)-alpha-D-GlcNAc-diphospho-di-trans,poly-cis-dolichol + GDP + H+.